{
  "term_id": "GO:2000562",
  "gene": "UniProtKB:B6A8C7",
  "term_label": "negative regulation of CD4-positive, alpha-beta T cell proliferation",
  "gene_symbol": "TARM1",
  "gene_name": "T-cell-interacting, activating receptor on myeloid cells protein 1"
}